{
  "term_id": "GO:0034089",
  "gene": "UniProtKB:Q9UJ98",
  "gene_name": "Cohesin subunit SA-3",
  "gene_symbol": "STAG3",
  "term_label": "establishment of meiotic sister chromatid cohesion"
}